{
  "gene_symbol": "FER1L6-AS1",
  "term_id": "UNKNOWN:0003",
  "gene": "UniProtKB:Q8NA97",
  "gene_name": "Putative uncharacterized protein FER1L6-AS1",
  "term_label": "Unknown cellular component"
}